{
  "gene": "UniProtKB:Q93083",
  "gene_name": "Metallothionein-1L",
  "term_label": "intracellular zinc ion homeostasis",
  "gene_symbol": "MT1L",
  "term_id": "GO:0006882"
}